saliva secretion [GO:0046541] (biological process) Also known as: salivation Regulation: regulated by GO:0046877; positively regulated by GO:0046878; negatively regulated by negative regulation of saliva secretion [GO:1905747] Sources: GOC:curators, UBERON:0001836 Relationships: is a type of body fluid secretion [GO:0007589]; is a type of GO:0022600; is a type of secretion by tissue [GO:0032941] Definition: The regulated release of saliva from the salivary glands. In man, the saliva is a turbid and slightly viscous fluid, generally of an alkaline reaction, and is secreted by the parotid, submaxillary, and sublingual glands. In the mouth the saliva is mixed with the secretion from the buccal glands. In man and many animals, saliva is an important digestive fluid on account of the presence of the peculiar enzyme, ptyalin.